2,3,4,5-tetrahydropyridine-2,6-dicarboxylate N-succinyltransferase activity [GO:0008666] (molecular function) Definition: Catalysis of the reaction: (S)-2,3,4,5-tetrahydrodipicolinate + H2O + succinyl-CoA = L-2-succinylamino-6-oxopimelate + CoA. Also known as: THDP N-succinyltransferase activity, succinyl-CoA:(S)-2,3,4,5-tetrahydropyridine-2,6-dicarboxylate N-succinyltransferase activity, succinyl-CoA:2,3,4,5-tetrahydropyridine-2,6-dicarboxylate N-succinyltransferase activity, succinyl-CoA:tetrahydrodipicolinate N-succinyltransferase activity, tetrahydrodipicolinate N-succinyltransferase activity, tetrahydrodipicolinate succinylase activity, tetrahydrodipicolinate succinyltransferase activity, tetrahydropicolinate succinylase activity Sources: EC:2.3.1.117, RHEA:17325 Relationships: is a type of GO:0016749